5-deoxy-D-glucuronate isomerase activity [GO:0102482] (molecular function) Sources: GOC:pz, RHEA:25840 Relationships: is a type of intramolecular oxidoreductase activity, interconverting aldoses and ketoses [GO:0016861] Definition: Catalysis of the reaction: 5-deoxy-D-glucuronate = 5-dehydro-2-deoxy-D-gluconate.